symbiont-mediated inactivation of host ribosome [GO:0141130] (biological process) References: PMID:1324134 Definition: A process in which a symbiont inhibits or disrupts translation of mRNA into protein in its host by inactivating its ribosomes. Relationships: is a type of symbiont-mediated suppression of host translation [GO:0039604] Also known as: symbiont-mediated host ribosome inactivation